{
  "term_id": "GO:0005544",
  "gene_name": "Annexin A3",
  "gene_symbol": "ANXA3",
  "gene": "UniProtKB:P12429",
  "term_label": "calcium-dependent phospholipid binding"
}